{
  "gene_name": "Protein canopy homolog 1",
  "gene_symbol": "CNPY1",
  "term_id": "UNKNOWN:0003",
  "gene": "UniProtKB:Q3B7I2",
  "term_label": "Unknown cellular component"
}